{
  "term_label": "transcription cis-regulatory region binding",
  "gene_symbol": "ZNF319",
  "gene_name": "Zinc finger protein 319",
  "gene": "UniProtKB:Q9P2F9",
  "term_id": "GO:0000976"
}